{
  "gene_name": "Fatty acyl-CoA reductase 2",
  "term_label": "alcohol-forming very long-chain fatty acyl-CoA reductase activity",
  "term_id": "GO:0080019",
  "gene": "UniProtKB:Q96K12",
  "gene_symbol": "FAR2"
}